dihydrosanguinarine 10-monooxygenase activity [GO:0047088] (molecular function) Definition: Catalysis of the reaction: dihydrosanguinarine + H+ + NADPH + O2 = 10-hydroxydihydrosanguinarine + H2O + NADP+. Sources: EC:1.14.14.100, RHEA:10528 Also known as: dihydrosanguinarine 10-hydroxylase activity, dihydrosanguinarine,NADPH:oxygen oxidoreductase (10-hydroxylating) Relationships: is a type of oxidoreductase activity, acting on paired donors, with incorporation or reduction of molecular oxygen, NAD(P)H as one donor, and incorporation of one atom of oxygen [GO:0016709]